{
  "term_id": "UNKNOWN:0002",
  "gene_name": "Putative postmeiotic segregation increased 2-like protein 1",
  "gene": "UniProtKB:A4D2B8",
  "gene_symbol": "PMS2P1",
  "term_label": "Unknown biological process"
}